{
  "gene": "UniProtKB:P51153",
  "gene_name": "Ras-related protein Rab-13",
  "term_label": "plasma membrane",
  "term_id": "GO:0005886",
  "gene_symbol": "RAB13"
}